epithelial cell proliferation [GO:0050673] (biological process) Subtypes: endothelial cell proliferation [GO:0001935], synoviocyte proliferation [GO:0002941], mammary gland epithelial cell proliferation [GO:0033598], GO:0043616, GO:0044342, urothelial cell proliferation [GO:0050674], Sertoli cell proliferation [GO:0060011], epithelial cell proliferation involved in lung morphogenesis [GO:0060502], GO:0060664, epithelial cell proliferation involved in prostate gland development [GO:0060767], GO:0072575, lens epithelial cell proliferation [GO:0097166], GO:0097325, sebum secreting cell proliferation [GO:1990654], cholangiocyte proliferation [GO:1990705], granulosa cell proliferation [GO:1990739], thyroid gland epithelial cell proliferation [GO:1990789], acinar cell proliferation [GO:1990863], epithelial cell proliferation involved in renal tubule morphogenesis [GO:2001013] Sources: ISBN:0721662544 Relationships: is_a GO:0008283 Definition: The multiplication or reproduction of epithelial cells, resulting in the expansion of a cell population. Epithelial cells make up the epithelium, the covering of internal and external surfaces of the body, including the lining of vessels and other small cavities. It consists of cells joined by small amounts of cementing substances. Regulation: regulated by GO:0050678; positively regulated by GO:0050679; RO_0002212 by GO:0050680